{
  "gene_symbol": "DMAP1",
  "gene": "UniProtKB:Q9NPF5",
  "term_label": "transcription corepressor activity",
  "term_id": "GO:0003714",
  "gene_name": "DNA methyltransferase 1-associated protein 1"
}